mRNA base-pairing post-transcriptional repressor activity [GO:1903231] (molecular function) Definition: A post-transcriptional repressor activity that acts by base-pairing with an mRNA to prevent gene expression. The binding can result in targeting the mRNA for degradation or interfering with mRNA translation resulting in post-transcriptional gene silencing. Also known as: mRNA base-pairing posttranscriptional repressor activity, mRNA binding involved in post-transcriptional gene silencing, mRNA binding involved in quelling, mRNA base-pairing translational repressor activity, translational inhibitor activity via mRNA base-pairing, mRNA binding involved in PTGS, mRNA binding involved in cosuppression, mRNA binding involved in posttranscriptional gene silencing, mRNA binding translation repressor activity Note: This term is intended for ncRNAs that act by base-pairing with a target mRNA. References: PMID:18197166, PMID:20533884 Sources: GOC:BHF, GOC:BHF_miRNA, GOC:ha, GOC:vw Relationships: is a type of GO:1990825; is part of regulatory ncRNA-mediated post-transcriptional gene silencing [GO:0035194]